induction of programmed cell death by ecdysone [GO:0035078] (biological process) Sources: GOC:bf Relationships: is a type of induction of programmed cell death by hormones [GO:0035081]; is part of response to ecdysone [GO:0035075] Definition: Any process induced by the steroid hormone 20-hydroxyecdysone (ecdysone) that directly activates any of the steps required for programmed cell death.